{
  "term_label": "Unknown biological process",
  "gene_name": "HCG2039775 (Fragment)",
  "gene": "UniProtKB:A0N4Z3",
  "gene_symbol": "TRAJ14",
  "term_id": "UNKNOWN:0002"
}